chloramphenicol transmembrane transport [GO:0042892] (biological process) References: PMID:29150447 Relationships: is a type of polyol transmembrane transport [GO:0015791]; is a type of amide transport [GO:0042886] Also known as: chloramphenicol transport Definition: The directed movement of chloramphenicol, a broad-spectrum antibiotic that inhibits bacterial protein synthesis, across a lipid bilayer, from one side of a membrane to the other.